atrioventricular node cell differentiation [GO:0060922] (BP) Sources: GOC:mtg_heart Relationships: is a type of cardiac septum cell differentiation [GO:0003292]; is a type of cardiac pacemaker cell differentiation [GO:0060920]; is part of atrioventricular node development [GO:0003162] Also known as: AV node cell differentiation Definition: The process in which a relatively unspecialized cell acquires specialized features of an atrioventricular (AV) node cell. AV node cells are pacemaker cells that are found in the atrioventricular node.